{
  "term_label": "cytoplasm",
  "term_id": "GO:0005737",
  "gene": "UniProtKB:O95067",
  "gene_name": "G2_mitotic-specific cyclin-B2",
  "gene_symbol": "CCNB2"
}